{
  "gene_name": "Kelch domain-containing protein 9",
  "term_id": "UNKNOWN:0003",
  "term_label": "Unknown cellular component",
  "gene": "UniProtKB:Q8NEP7",
  "gene_symbol": "KLHDC9"
}